{
  "term_label": "regulation of actin cytoskeleton organization",
  "gene": "UniProtKB:Q68EM7",
  "term_id": "GO:0032956",
  "gene_name": "Rho GTPase-activating protein 17",
  "gene_symbol": "ARHGAP17"
}